{
  "term_id": "GO:0007015",
  "gene_name": "Transgelin-3",
  "gene_symbol": "TAGLN3",
  "gene": "UniProtKB:Q9UI15",
  "term_label": "actin filament organization"
}